pre-snoRNP complex [GO:0070761] (cellular component) References: PMID:17636026, PMID:17709390 Sources: GOC:BHF, GOC:mah, GOC:rl Definition: A ribonucleoprotein complex that contains a precursor small nucleolar RNA (pre-snoRNA) and associated proteins, and forms during small nucleolar ribonucleoprotein complex (snoRNP) assembly. Pre-snoRNP complexes may contain proteins not found in the corresponding mature snoRNP complexes. Also known as: pre-small nucleolar ribonucleoprotein complex Relationships: is a type of ribonucleoprotein complex [GO:1990904]